{
  "gene": "UniProtKB:Q15072",
  "gene_symbol": "ZNF146",
  "gene_name": "Zinc finger protein OZF",
  "term_label": "nucleus",
  "term_id": "GO:0005634"
}